{
  "gene_name": "Myelin protein P0",
  "gene_symbol": "MPZ",
  "term_label": "plasma membrane",
  "term_id": "GO:0005886",
  "gene": "UniProtKB:P25189"
}